queuosine nucleosidase activity [GO:0106432] (molecular function) Definition: Catalysis of the reaction: queuosine 5'-phosphate + H2O = queuine + D-ribose 5-phosphate. References: PMID:35940128 Sources: RHEA:75387 Also known as: queuosine nucleoside glycosylase, tRNA queuosine nucleoside glycosylase Relationships: is_a purine nucleosidase activity [GO:0008477]